{
  "gene": "UniProtKB:Q9BV99",
  "gene_name": "Leucine-rich repeat-containing protein 61",
  "term_id": "UNKNOWN:0002",
  "gene_symbol": "LRRC61",
  "term_label": "Unknown biological process"
}